negative regulation of pseudopodium assembly [GO:0031273] (biological process) Definition: Any process that stops, prevents, or reduces the frequency, rate or extent of the assembly of pseudopodia. Also known as: inhibition of pseudopodium formation, down regulation of pseudopodium formation, down-regulation of pseudopodium formation, downregulation of pseudopodium formation, negative regulation of pseudopodium formation Relationships: is a type of regulation of pseudopodium assembly [GO:0031272]; is a type of negative regulation of plasma membrane bounded cell projection assembly [GO:0120033]; negatively regulates pseudopodium assembly [GO:0031269] Sources: GOC:pg